plastid mRNA editing complex [GO:0031020] (cellular component) Relationships: is_a mRNA editing complex [GO:0045293]; BFO_0000050 plastid [GO:0009536] Sources: GOC:mah Definition: An mRNA editing complex found in a plastid. Also known as: plastid editosome